chemosynthesis [GO:0062097] (biological process) References: PMID:25050523 Relationships: is a type of GO:0008152 Definition: The cellular metabolic process in which organic chemical compounds are synthesized from carbon-containing molecules and nutrients using energy obtained from the oxidation of inorganic compounds or methane.